{
  "term_id": "GO:0071805",
  "gene": "UniProtKB:Q6UVM3",
  "gene_symbol": "KCNT2",
  "term_label": "potassium ion transmembrane transport",
  "gene_name": "Potassium channel subfamily T member 2"
}